D-alanine-D-alanine ligase activity [GO:0008716] (molecular function) Definition: Catalysis of the reaction: 2 D-alanine + ATP = D-alanyl-D-alanine + ADP + 2 H+ + phosphate. Sources: EC:6.3.2.4, RHEA:11224 Also known as: D-Ala-D-Ala synthetase activity, D-alanine:D-alanine ligase (ADP-forming), D-alanyl-D-alanine synthetase activity, D-alanylalanine synthetase activity, alanine:alanine ligase (ADP-forming) activity, alanylalanine synthetase activity Relationships: is a type of acid-amino acid ligase activity [GO:0016881]